{
  "term_label": "olfactory receptor activity",
  "gene": "UniProtKB:P47881",
  "gene_name": "Olfactory receptor 3A1",
  "gene_symbol": "OR3A1",
  "term_id": "GO:0004984"
}